{
  "gene_name": "E3 ubiquitin-protein ligase RLIM",
  "term_label": "nucleus",
  "term_id": "GO:0005634",
  "gene": "UniProtKB:Q9NVW2",
  "gene_symbol": "RLIM"
}